{
  "gene_symbol": "ZP3",
  "term_label": "egg coat",
  "term_id": "GO:0035805",
  "gene_name": "Zona pellucida sperm-binding protein 3",
  "gene": "UniProtKB:P21754"
}